{
  "gene": "UniProtKB:Q9P2J2",
  "term_label": "cell-cell adhesion mediator activity",
  "term_id": "GO:0098632",
  "gene_symbol": "IGSF9",
  "gene_name": "Protein turtle homolog A"
}